synaptic signaling via neuropeptide [GO:0099538] (biological process) Relationships: is_a synaptic signaling [GO:0099536] Subtypes: trans-synaptic signaling by neuropeptide [GO:0099540] Sources: GOC:dos Definition: Cell-cell signaling to or from a synapse, mediated by a peptide.